{
  "gene_name": "C-C chemokine receptor type 7",
  "term_id": "GO:0009897",
  "gene_symbol": "CCR7",
  "gene": "UniProtKB:P32248",
  "term_label": "external side of plasma membrane"
}